{
  "term_label": "endoderm formation",
  "term_id": "GO:0001706",
  "gene": "UniProtKB:Q05923",
  "gene_name": "Dual specificity protein phosphatase 2",
  "gene_symbol": "DUSP2"
}